{
  "term_label": "voltage-gated calcium channel activity",
  "gene": "UniProtKB:Q8NEC5",
  "term_id": "GO:0005245",
  "gene_symbol": "CATSPER1",
  "gene_name": "Cation channel sperm-associated protein 1"
}